{
  "term_id": "GO:0005654",
  "gene_symbol": "NOC2L",
  "gene": "UniProtKB:Q9Y3T9",
  "gene_name": "Nucleolar complex protein 2 homolog",
  "term_label": "nucleoplasm"
}